{
  "gene_name": "Protein delta homolog 1",
  "term_id": "UNKNOWN:0001",
  "term_label": "Unknown molecular function",
  "gene_symbol": "DLK1",
  "gene": "UniProtKB:P80370"
}